negative regulation of toll-like receptor 5 signaling pathway [GO:0034148] (biological process) Definition: Any process that stops, prevents, or reduces the frequency, rate, or extent of toll-like receptor 5 signaling pathway. References: PMID:16551253, PMID:17328678 Sources: GOC:add Also known as: negative regulation of TLR5 signaling pathway, negative regulation of toll-like receptor 5 signalling pathway Relationships: is a type of negative regulation of immune system process [GO:0002683]; is_a negative regulation of signal transduction [GO:0009968]; is a type of regulation of toll-like receptor 5 signaling pathway [GO:0034147]; negatively regulates toll-like receptor 5 signaling pathway [GO:0034146]